{
  "gene_name": "V-type proton ATPase subunit S1",
  "term_label": "Unknown molecular function",
  "gene_symbol": "ATP6AP1",
  "term_id": "UNKNOWN:0001",
  "gene": "UniProtKB:Q15904"
}